{
  "term_label": "postsynaptic recycling endosome",
  "gene_name": "Ras-related protein Rab-11A",
  "gene_symbol": "RAB11A",
  "gene": "UniProtKB:P62491",
  "term_id": "GO:0098837"
}